cellular response to acadesine [GO:1904102] (biological process) References: PMID:20802119 Sources: GOC:TermGenie, GOC:mr, GO_REF:0000071 Relationships: is a type of cellular response to nitrogen compound [GO:1901699]; is a type of cellular response to oxygen-containing compound [GO:1901701]; is a type of response to acadesine [GO:1904101] Definition: Any process that results in a change in state or activity of a cell (in terms of movement, secretion, enzyme production, gene expression, etc.) as a result of an acadesine stimulus.